positive regulation of spindle checkpoint [GO:0090232] (biological process) Sources: GOC:ascb_2009, GOC:dph, GOC:tb Also known as: spindle checkpoint activation Subtypes: positive regulation of mitotic cell cycle spindle assembly checkpoint [GO:0090267], GO:1905326 Definition: Any process that increases the rate, frequency, or extent of the spindle checkpoint, a cell cycle checkpoint that delays the metaphase/anaphase transition until the spindle is correctly assembled and oriented, and chromosomes are attached to the spindle. Relationships: is a type of regulation of spindle checkpoint [GO:0090231]; is a type of positive regulation of cell cycle checkpoint [GO:1901978]; positively regulates spindle checkpoint signaling [GO:0031577]